{
  "term_label": "bicellular tight junction assembly",
  "gene_symbol": "POF1B",
  "gene_name": "Protein POF1B",
  "gene": "UniProtKB:Q8WVV4",
  "term_id": "GO:0070830"
}